{
  "term_label": "actin filament bundle organization",
  "gene_symbol": "RFLNB",
  "term_id": "GO:0061572",
  "gene": "UniProtKB:Q8N5W9",
  "gene_name": "Refilin-B"
}